{
  "term_label": "Unknown biological process",
  "gene": "UniProtKB:Q6ZSJ8",
  "gene_symbol": "C1orf122",
  "gene_name": "Uncharacterized protein C1orf122",
  "term_id": "UNKNOWN:0002"
}